{
  "gene": "UniProtKB:O75900",
  "gene_symbol": "MMP23B",
  "gene_name": "Matrix metalloproteinase-23",
  "term_label": "extracellular matrix organization",
  "term_id": "GO:0030198"
}